{
  "gene_symbol": "MEGF10",
  "gene_name": "Multiple epidermal growth factor-like domains protein 10",
  "term_label": "engulfment of apoptotic cell",
  "term_id": "GO:0043652",
  "gene": "UniProtKB:Q96KG7"
}